{
  "gene_symbol": "FAM161A",
  "term_label": "cilium organization",
  "term_id": "GO:0044782",
  "gene_name": "Protein FAM161A",
  "gene": "UniProtKB:Q3B820"
}